{
  "term_label": "Unknown molecular function",
  "gene_name": "Coiled-coil domain-containing protein 74B",
  "gene": "UniProtKB:Q96LY2",
  "gene_symbol": "CCDC74B",
  "term_id": "UNKNOWN:0001"
}